{
  "gene_symbol": "SLC4A1",
  "gene_name": "Band 3 anion transport protein",
  "term_id": "GO:0005886",
  "gene": "UniProtKB:P02730",
  "term_label": "plasma membrane"
}